glucuronosyl-N-acetylglucosaminyl-proteoglycan 4-alpha-N-acetylglucosaminyltransferase activity [GO:0050508] (molecular function) Sources: EC:2.4.1.224, MetaCyc:2.4.1.224-RXN, RHEA:16213 Relationships: is a type of acetylglucosaminyltransferase activity [GO:0008375] Definition: Catalysis of the reaction: 3-O-{[(1->4)-beta-D-GlcA-(1->4)-alpha-D-GlcNAc](n)-(1->4)-beta-D-GlcA-(1->3)-beta-D-Gal-(1->3)-beta-D-Gal-(1->4)-beta-D-Xyl}-L-seryl-[protein] + UDP-N-acetyl-alpha-D-glucosamine = 3-O-{alpha-D-GlcNAc-[(1->4)-beta-D-GlcA-(1->4)-alpha-D-GlcNAc](n)-(1->4)-beta-D-GlcA-(1->3)-beta-D-Gal-(1->3)-beta-D-Gal-(1->4)-beta-D-Xyl}-L-seryl-[protein] + H+ + UDP. Also known as: glucuronosyl-N-acetylglucosaminyl-proteoglycan 4-a-N-acetylglucosaminyltransferase activity, UDP-N-acetyl-D-glucosamine:beta-D-glucuronosyl-(1->4)-N-acetyl-alpha-D-glucosaminyl-proteoglycan 4-alpha-N-acetylglucosaminyltransferase activity, alpha-N-acetylglucosaminyltransferase II activity, glucuronyl-N-acetylglucosaminylproteoglycan alpha-1,4-N-acetylglucosaminyltransferase activity